{
  "term_id": "UNKNOWN:0003",
  "gene": "UniProtKB:Q8NC54",
  "gene_symbol": "KCT2",
  "term_label": "Unknown cellular component",
  "gene_name": "Keratinocyte-associated transmembrane protein 2"
}